bone regeneration [GO:1990523] (biological process) References: PMID:25257467 Relationships: is a type of tissue regeneration [GO:0042246] Definition: The regrowth of bone following its loss or destruction.